cell growth involved in growth plate cartilage chondrocyte morphogenesis [GO:0003432] (biological process) Relationships: is a type of growth plate cartilage chondrocyte growth [GO:0003430]; is part of growth plate cartilage chondrocyte morphogenesis [GO:0003429] Sources: GOC:ascb_2009, GOC:dph, GOC:tb Definition: The growth of a growth plate cartilage chondrocyte, where growth contributes to the shaping of the chondrocyte over time.